{
  "term_label": "Unknown molecular function",
  "gene": "UniProtKB:Q969X5",
  "term_id": "UNKNOWN:0001",
  "gene_symbol": "ERGIC1",
  "gene_name": "Endoplasmic reticulum-Golgi intermediate compartment protein 1"
}